DNA polymerase processivity factor complex [GO:0044796] (cellular component) Definition: A protein complex which is capable of increasing the processivity of nucleotide polymerization by DNA polymerase as a part of DNA replication. Sources: GOC:bhm, GOC:jl Relationships: is a type of enzyme activator complex [GO:0150005] Subtypes: GO:0043626, DNA polymerase III, beta sliding clamp processivity factor complex [GO:0044775]